{
  "term_label": "inflammatory response",
  "term_id": "GO:0006954",
  "gene": "UniProtKB:P16619",
  "gene_name": "C-C motif chemokine 3-like 1",
  "gene_symbol": "CCL3L1"
}